{
  "gene": "UniProtKB:P17535",
  "gene_name": "Transcription factor JunD",
  "gene_symbol": "JUND",
  "term_label": "regulation of cell population proliferation",
  "term_id": "GO:0042127"
}